regulation of fatty acid transport [GO:2000191] (biological process) Relationships: is a type of regulation of lipid transport [GO:0032368]; is a type of GO:0032890; regulates GO:0015908 Sources: GOC:BHF Subtypes: GO:0032303, GO:0140212, negative regulation of fatty acid transport [GO:2000192], positive regulation of fatty acid transport [GO:2000193] Definition: Any process that modulates the frequency, rate or extent of fatty acid transport.